{
  "term_id": "GO:0030126",
  "term_label": "COPI vesicle coat",
  "gene_symbol": "COPZ1",
  "gene": "UniProtKB:P61923",
  "gene_name": "Coatomer subunit zeta-1"
}